regulation of complement-dependent cytotoxicity [GO:1903659] (BP) Relationships: is a type of regulation of cell killing [GO:0031341]; regulates complement-dependent cytotoxicity [GO:0097278] References: PMID:24280217 Sources: GOC:TermGenie, GO_REF:0000058 Subtypes: negative regulation of complement-dependent cytotoxicity [GO:1903660], positive regulation of complement-dependent cytotoxicity [GO:1903661] Definition: Any process that modulates the frequency, rate or extent of complement-dependent cytotoxicity.